cell division [GO:0051301] (biological process) Subtypes: growth plate cartilage chondrocyte division [GO:0003423], GO:0007114, spermatogonial cell division [GO:0007284], asymmetric cell division [GO:0008356], epidermal cell division [GO:0010481], myoblast division [GO:0014872], stem cell division [GO:0017145], schizogony [GO:0020014], forebrain ventricular zone progenitor cell division [GO:0021869], radial glial cell division in pallium [GO:0022015], embryonic cleavage [GO:0040016], spermatocyte division [GO:0048137], glioblast division [GO:0048860], GO:0055057, GO:0090510, periclinal cell division [GO:0090511], GO:0098725, GO:0110069 Relationships: is a type of cellular process [GO:0009987] Sources: GOC:di, GOC:go_curators, GOC:pr Definition: The process resulting in division and partitioning of components of a cell to form more cells; may or may not be accompanied by the physical separation of a cell into distinct, individually membrane-bounded daughter cells. Regulation: regulated by regulation of cell division [GO:0051302]; positively regulated by positive regulation of cell division [GO:0051781]; negatively regulated by negative regulation of cell division [GO:0051782] Note: Note that this term differs from 'cytokinesis ; GO:0000910' in that cytokinesis does not include nuclear division.